{
  "term_label": "GABA-A receptor activity",
  "gene": "UniProtKB:P28472",
  "gene_symbol": "GABRB3",
  "term_id": "GO:0004890",
  "gene_name": "Gamma-aminobutyric acid receptor subunit beta-3"
}